regulation of keratinocyte apoptotic process [GO:1902172] (biological process) References: PMID:18938133 Sources: GOC:BHF, GOC:TermGenie, GOC:mtg_apoptosis, GOC:rl Relationships: is a type of regulation of epithelial cell apoptotic process [GO:1904035]; regulates keratinocyte apoptotic process [GO:0097283] Definition: Any process that modulates the frequency, rate or extent of keratinocyte apoptotic process. Subtypes: negative regulation of keratinocyte apoptotic process [GO:1902173], positive regulation of keratinocyte apoptotic process [GO:1902174] Also known as: regulation of keratinocyte apoptosis